{
  "gene_symbol": "AQR",
  "term_label": "mRNA binding",
  "term_id": "GO:0003729",
  "gene": "UniProtKB:O60306",
  "gene_name": "RNA helicase aquarius"
}